{
  "term_label": "Unknown cellular component",
  "gene": "UniProtKB:O15294",
  "gene_symbol": "OGT",
  "gene_name": "UDP-N-acetylglucosamine--peptide N-acetylglucosaminyltransferase 110 kDa subunit",
  "term_id": "UNKNOWN:0003"
}